{
  "gene_name": "RUN and FYVE domain-containing protein 1",
  "gene": "UniProtKB:Q96T51",
  "term_label": "protein transport",
  "term_id": "GO:0015031",
  "gene_symbol": "RUFY1"
}